{
  "term_label": "ubiquitin-like ligase-substrate adaptor activity",
  "gene_name": "F-box only protein 48",
  "gene": "UniProtKB:Q5FWF7",
  "term_id": "GO:1990756",
  "gene_symbol": "FBXO48"
}